{
  "gene": "UniProtKB:Q9HBX8",
  "gene_name": "Leucine-rich repeat-containing G-protein coupled receptor 6",
  "gene_symbol": "LGR6",
  "term_label": "Roundabout binding",
  "term_id": "GO:0048495"
}